{
  "term_id": "GO:0005786",
  "term_label": "signal recognition particle, endoplasmic reticulum targeting",
  "gene": "UniProtKB:P61011",
  "gene_symbol": "SRP54",
  "gene_name": "Signal recognition particle subunit SRP54"
}